{
  "term_id": "GO:0030296",
  "gene": "UniProtKB:Q02297",
  "gene_symbol": "NRG1",
  "term_label": "protein tyrosine kinase activator activity",
  "gene_name": "Pro-neuregulin-1, membrane-bound isoform"
}